intracellular triglyceride homeostasis [GO:0035356] (biological process) Definition: A homeostatic process involved in the maintenance of a steady state level of triglyceride within a cell. Sources: GOC:BHF Also known as: cellular triglyceride homeostasis Relationships: is a type of intracellular chemical homeostasis [GO:0055082]; is a type of triglyceride homeostasis [GO:0070328]